{
  "term_id": "GO:0003823",
  "gene": "UniProtKB:A0A075B7B6",
  "term_label": "antigen binding",
  "gene_symbol": "IGHV4OR15-8",
  "gene_name": "Immunoglobulin heavy variable 4_OR15-8 (non-functional) (Fragment)"
}